adenylylsulfatase activity [GO:0047627] (molecular function) Definition: Catalysis of the reaction: 5'-adenylyl sulfate + H2O = AMP + 2 H+ + sulfate. Also known as: adenylylsulphatase activity, adenosine 5-phosphosulfate sulfohydrolase activity, adenylylsulfate sulfohydrolase activity Relationships: is a type of hydrolase activity, acting on acid anhydrides, in sulfonyl-containing anhydrides [GO:0016819] Sources: EC:3.6.2.1, RHEA:17041